dimethylmaleate hydratase activity [GO:0047868] (molecular function) Definition: Catalysis of the reaction: (2R,3S)-2,3-dimethylmalate = dimethylmaleate + H2O. Sources: EC:4.2.1.85, RHEA:20253 Also known as: (2R,3S)-2,3-dimethylmalate hydro-lyase (dimethylmaleate-forming), (2R,3S)-2,3-dimethylmalate hydro-lyase activity Relationships: is a type of hydro-lyase activity [GO:0016836]